{
  "term_id": "GO:0051660",
  "term_label": "establishment of centrosome localization",
  "gene": "UniProtKB:Q9Y592",
  "gene_name": "Centrosomal protein of 83 kDa",
  "gene_symbol": "CEP83"
}